anterior lateral line nerve glial cell development [GO:0048939] (biological process) Definition: The process aimed at the progression of a glial cell in the anterior lateral line nerve over time, from initial commitment of the cell to a specific fate, to the fully functional differentiated cell. Sources: GOC:dgh Relationships: is a type of lateral line nerve glial cell development [GO:0048937]; BFO_0000050 anterior lateral line nerve glial cell differentiation [GO:0048913]